{
  "gene_symbol": "C16orf78",
  "gene": "UniProtKB:Q8WTQ4",
  "term_id": "UNKNOWN:0001",
  "gene_name": "Uncharacterized protein C16orf78",
  "term_label": "Unknown molecular function"
}